trihydroxypterocarpan dimethylallyltransferase activity [GO:0047292] (molecular function) Sources: EC:2.5.1.36 Definition: Catalysis of the reaction: (6AS,11AS)-3,6A,9-trihydroxypterocarpan + dimethylallyl-pyrophosphate = glyceollin + diphosphate. Relationships: is a type of GO:0016765 Also known as: dimethylallyl-diphosphate:(6aS,11aS)-3,6a,9-trihydroxypterocarpan dimethylallyltransferase activity, dimethylallyl-diphosphate:(6aS,11aS)-3,6a,9-trihydroxypterocarpan dimethyltransferase activity, dimethylallylpyrophosphate:3,6a,9-trihydroxypterocarpan dimethylallyltransferase activity, dimethylallylpyrophosphate:trihydroxypterocarpan dimethylallyl transferase activity